tri-(coumaroyl or caffeoyl) spermidine meta-hydroxylase activity [GO:0072533] (molecular function) Note: Note that the overall reaction representing three successive executions of this activity is N1,N5,N10-tricoumaroyl spermidine + 3 NADPH + 3 O2 = N1,N5,N10-tricaffeoyl spermidine + 3 NADP+ + 3 H2O; this corresponds to the MetaCyc reaction RXN-11260 (http://biocyc.org/META/NEW-IMAGE?type=REACTION&object=RXN-11260). Relationships: is a type of oxidoreductase activity, acting on paired donors, with incorporation or reduction of molecular oxygen, NAD(P)H as one donor, and incorporation of one atom of oxygen [GO:0016709] References: PMID:19779199 Sources: GOC:kad Definition: Catalysis of the meta-hydroxylation of any of the three phenolic rings on tricoumaroyl spermidine or any of its mono- or dicaffeoyl spermidine derivatives. Subtypes: tricoumaroylspermidine meta-hydroxylase activity [GO:0072547], dicoumaroyl monocaffeoyl spermidine meta-hydroxylase activity [GO:0072548], monocoumaroyl dicaffeoyl spermidine meta-hydroxylase activity [GO:0072549]